{
  "gene": "UniProtKB:P52954",
  "gene_name": "Transcription factor LBX1",
  "gene_symbol": "LBX1",
  "term_label": "nucleus",
  "term_id": "GO:0005634"
}